{
  "term_id": "GO:0009986",
  "term_label": "cell surface",
  "gene": "UniProtKB:A6NJW9",
  "gene_name": "T-cell surface glycoprotein CD8 beta-2 chain",
  "gene_symbol": "CD8B2"
}